{
  "gene_symbol": "DAB2IP",
  "term_id": "GO:1902531",
  "gene_name": "Disabled homolog 2-interacting protein",
  "term_label": "regulation of intracellular signal transduction",
  "gene": "UniProtKB:Q5VWQ8"
}